{
  "term_id": "GO:0005770",
  "term_label": "late endosome",
  "gene_name": "Multivesicular body subunit 12B",
  "gene_symbol": "MVB12B",
  "gene": "UniProtKB:Q9H7P6"
}